{
  "term_id": "GO:0019782",
  "gene": "UniProtKB:P41226",
  "term_label": "ISG15 activating enzyme activity",
  "gene_symbol": "UBA7",
  "gene_name": "Ubiquitin-like modifier-activating enzyme 7"
}